{
  "gene_name": "Putative olfactory receptor 8G2",
  "term_id": "UNKNOWN:0003",
  "term_label": "Unknown cellular component",
  "gene_symbol": "OR8G2P",
  "gene": "UniProtKB:Q6IF36"
}